{
  "term_id": "GO:0016020",
  "term_label": "membrane",
  "gene_name": "Transmembrane 4 L6 family member 20",
  "gene": "UniProtKB:Q53R12",
  "gene_symbol": "TM4SF20"
}